{
  "term_id": "GO:0031012",
  "gene_symbol": "COMP",
  "gene": "UniProtKB:P49747",
  "term_label": "extracellular matrix",
  "gene_name": "Cartilage oligomeric matrix protein"
}